{
  "term_id": "GO:0005829",
  "gene_symbol": "PPP2R5A",
  "gene_name": "Serine_threonine-protein phosphatase 2A 56 kDa regulatory subunit alpha isoform",
  "term_label": "cytosol",
  "gene": "UniProtKB:Q15172"
}